{
  "gene_name": "dCTP pyrophosphatase 1",
  "term_label": "DNA protection",
  "gene": "UniProtKB:Q9H773",
  "gene_symbol": "DCTPP1",
  "term_id": "GO:0042262"
}